{
  "term_label": "Unknown cellular component",
  "gene": "UniProtKB:Q86WA6",
  "term_id": "UNKNOWN:0003",
  "gene_name": "Valacyclovir hydrolase",
  "gene_symbol": "BPHL"
}